mature B cell differentiation [GO:0002335] (biological process) Sources: GOC:jal, ISBN:0781735149 Subtypes: GO:0001923, GO:0002313 Also known as: mature B lymphocyte differentiation, mature B-cell differentiation, mature B-lymphocyte differentiation, mature cell development Definition: The process in which transitional stage B cells acquire the specialized features of mature B cells in the spleen. Note: Note that immunologists typically use the word 'development' to refer to cells of B or T cell lineages undergoing the process that GO describes as 'cell differentiation'. Relationships: is a type of GO:0030183